2-iminoacetate synthase complex [GO:1902508] (CC) References: PMID:12650933 Sources: GOC:TermGenie, GOC:bhm Also known as: ThiH-ThiG complex Relationships: is a type of GO:1902494 Definition: A protein complex which is capable of 2-iminoacetate synthase activity.